{
  "gene_name": "Metallothionein-1L",
  "term_id": "GO:0005737",
  "gene": "UniProtKB:Q93083",
  "term_label": "cytoplasm",
  "gene_symbol": "MT1L"
}